{
  "gene_symbol": "DENND2B",
  "term_id": "UNKNOWN:0003",
  "gene_name": "DENN domain-containing protein 2B",
  "gene": "UniProtKB:P78524",
  "term_label": "Unknown cellular component"
}